{
  "term_label": "signaling receptor binding",
  "gene": "UniProtKB:Q9UKU9",
  "term_id": "GO:0005102",
  "gene_name": "Angiopoietin-related protein 2",
  "gene_symbol": "ANGPTL2"
}